{
  "term_label": "extracellular space",
  "gene": "UniProtKB:O14669",
  "term_id": "GO:0005615",
  "gene_symbol": "PRRG2",
  "gene_name": "Transmembrane gamma-carboxyglutamic acid protein 2"
}